{
  "gene_symbol": "GPHB5",
  "term_label": "G protein-coupled receptor signaling pathway",
  "gene_name": "Glycoprotein hormone beta-5",
  "term_id": "GO:0007186",
  "gene": "UniProtKB:Q86YW7"
}